positive regulation of melanosome transport [GO:1902910] (biological process) References: PMID:23334344 Sources: GOC:TermGenie, GOC:als, GO_REF:0000058 Relationships: is a type of positive regulation of cellular process [GO:0048522]; is_a positive regulation of transport [GO:0051050]; is a type of regulation of melanosome transport [GO:1902908]; positively regulates GO:0032402 Definition: Any process that activates or increases the frequency, rate or extent of melanosome transport. Also known as: up regulation of melanosome transport, up-regulation of melanosome transport, upregulation of melanosome transport, activation of melanosome transport